{
  "gene": "UniProtKB:Q9BXL6",
  "gene_name": "Caspase recruitment domain-containing protein 14",
  "gene_symbol": "CARD14",
  "term_label": "signal transduction",
  "term_id": "GO:0007165"
}